{
  "gene": "UniProtKB:Q8N556",
  "gene_symbol": "AFAP1",
  "term_id": "GO:0005884",
  "term_label": "actin filament",
  "gene_name": "Actin filament-associated protein 1"
}